has_synonym_type [oboInOwl#hasSynonymType]